{
  "gene_name": "Unconventional myosin-Ig",
  "term_label": "actin filament-based movement",
  "gene": "UniProtKB:B0I1T2",
  "gene_symbol": "MYO1G",
  "term_id": "GO:0030048"
}